detection of abiotic stimulus [GO:0009582] (biological process) Subtypes: detection of light stimulus [GO:0009583], detection of gravity [GO:0009590], GO:0016048, GO:0043575, detection of electrical stimulus [GO:0050981], detection of mechanical stimulus [GO:0050982], detection of humidity [GO:0098513] Relationships: is a type of response to abiotic stimulus [GO:0009628]; is a type of detection of stimulus [GO:0051606] Sources: GOC:hb Also known as: perception of abiotic stimulus Definition: The series of events in which an (non-living) abiotic stimulus is received by a cell and converted into a molecular signal.